transmembrane receptor protein tyrosine kinase inhibitor activity [GO:0030293] (molecular function) Sources: GOC:mah Relationships: is a type of protein tyrosine kinase inhibitor activity [GO:0030292]; is a type of signaling receptor inhibitor activity [GO:0030547]; negatively regulates transmembrane receptor protein tyrosine kinase activity [GO:0004714] Definition: Binds to and stops, prevents or reduces the activity of a transmembrane receptor protein tyrosine kinase.